embryonic pattern specification [GO:0009880] (biological process) Subtypes: GO:0000578, somite specification [GO:0001757], blastoderm segmentation [GO:0007350], terminal region determination [GO:0007362] Sources: GOC:go_curators, ISBN:0521436125 Relationships: is a type of pattern specification process [GO:0007389]; is part of GO:0009790 Also known as: embryonic pattern biosynthesis, embryonic pattern formation, ventral/lateral system Regulation: regulated by regulation of embryonic pattern specification [GO:1902875]; negatively regulated by negative regulation of embryonic pattern specification [GO:1902876]; positively regulated by positive regulation of embryonic pattern specification [GO:1902877] Definition: The process that results in the patterns of cell differentiation that will arise in an embryo.